{
  "gene": "UniProtKB:O00233",
  "gene_symbol": "PSMD9",
  "term_id": "GO:0005737",
  "term_label": "cytoplasm",
  "gene_name": "26S proteasome non-ATPase regulatory subunit 9"
}